labial disc development [GO:0035217] (biological process) Definition: Progression of the labial imaginal disc over time, from its initial formation through to its metamorphosis to form adult structures including parts of the proboscis. Sources: GOC:bf, ISBN:0879694238 Relationships: is a type of imaginal disc development [GO:0007444]